{
  "gene_symbol": "CCM2L",
  "term_label": "heart morphogenesis",
  "gene_name": "Cerebral cavernous malformations 2 protein-like",
  "term_id": "GO:0003007",
  "gene": "UniProtKB:Q9NUG4"
}